{
  "term_label": "Unknown biological process",
  "gene_symbol": "CFAP91",
  "gene": "UniProtKB:Q7Z4T9",
  "term_id": "UNKNOWN:0002",
  "gene_name": "Cilia- and flagella-associated protein 91"
}